{
  "gene_name": "Serine_threonine-protein kinase BRSK1",
  "gene_symbol": "BRSK1",
  "term_label": "tau-protein kinase activity",
  "term_id": "GO:0050321",
  "gene": "UniProtKB:Q8TDC3"
}